{
  "gene_symbol": "C1QTNF4",
  "term_label": "positive regulation of interleukin-6-mediated signaling pathway",
  "gene": "UniProtKB:Q9BXJ3",
  "gene_name": "Complement C1q tumor necrosis factor-related protein 4",
  "term_id": "GO:0070105"
}